nicotinamide riboside hydrolase activity [GO:0070635] (molecular function) Relationships: is a type of hydrolase activity, hydrolyzing N-glycosyl compounds [GO:0016799] Definition: Catalysis of the reaction: nicotinamide riboside + H2O = nicotinamide + D-ribose. Also known as: N-ribosylnicotinamide hydrolase activity, nicotinamide ribonucleoside hydrolase activity References: PMID:19001417 Sources: MetaCyc:RXN-8441